{
  "gene": "UniProtKB:Q9P2K6",
  "gene_name": "Kelch-like protein 42",
  "term_id": "UNKNOWN:0001",
  "term_label": "Unknown molecular function",
  "gene_symbol": "KLHL42"
}